{
  "gene_name": "Olfactory receptor 8B8",
  "gene": "UniProtKB:Q15620",
  "term_label": "sensory perception of smell",
  "gene_symbol": "OR8B8",
  "term_id": "GO:0007608"
}